symbiont-mediated perturbation of host signal transduction pathway [GO:0052027] (biological process) Definition: A process in which a symbiont alters or subverts a signal transduction pathway in its host organism. The host is defined as the larger of the organisms involved in a symbiotic interaction. Sources: GOC:mtg_pamgo_17jul06 Also known as: modulation of signal transduction in other organism involved in symbiotic interaction, modulation by symbiont of host signal transduction pathway, modulation of host signal transduction by symbiont, perturbation of host signal transduction pathway, regulation by symbiont of host signal transduction pathway, modulation by symbiont of host signal transduction Relationships: is a type of symbiont-mediated perturbation of host cellular process [GO:0044068] Subtypes: GO:0044082, symbiont-mediated activation of host signal transduction pathway [GO:0052028], symbiont-mediated suppression of host signal transduction pathway [GO:0052029], symbiont-mediated perturbation of host MAPK cascade [GO:0052080], GO:0052081, symbiont-mediated perturbation of host jasmonic acid signaling [GO:0052088], GO:0075109, symbiont-mediated perturbation of host NF-kappaB cascade [GO:0085032], symbiont-mediated cAMP intoxication of host cell [GO:0141042]